endobrevin-SNAP-25-syntaxin-2 complex [GO:0070049] (cellular component) Also known as: SNARE complex (Stx2, Snap25, Vamp8), Stx2-Snap25-Vamp8 complex Definition: A SNARE complex that contains endobrevin (VAMP8), SNAP-25, and syntaxin 2 (or orthologs thereof). References: PMID:10336434 Relationships: is a type of GO:0031201